{
  "gene": "UniProtKB:P04114",
  "gene_name": "Apolipoprotein B-100",
  "gene_symbol": "APOB",
  "term_id": "GO:0034362",
  "term_label": "low-density lipoprotein particle"
}